{
  "gene_name": "Receptor-type tyrosine-protein phosphatase H",
  "gene_symbol": "PTPRH",
  "gene": "UniProtKB:Q9HD43",
  "term_id": "GO:0007411",
  "term_label": "axon guidance"
}